{
  "term_id": "GO:0001227",
  "term_label": "DNA-binding transcription repressor activity, RNA polymerase II-specific",
  "gene": "UniProtKB:Q9HCK0",
  "gene_symbol": "ZBTB26",
  "gene_name": "Zinc finger and BTB domain-containing protein 26"
}